response to glucose [GO:0009749] (biological process) Also known as: response to glucose stimulus Definition: Any process that results in a change in state or activity of a cell or an organism (in terms of movement, secretion, enzyme production, gene expression, etc.) as a result of a glucose stimulus. Sources: GOC:jl Relationships: is a type of response to hexose [GO:0009746] Subtypes: GO:0051594, cellular response to glucose stimulus [GO:0071333]